{
  "gene_symbol": "ZNF536",
  "gene": "UniProtKB:O15090",
  "term_id": "GO:0006355",
  "gene_name": "Zinc finger protein 536",
  "term_label": "regulation of DNA-templated transcription"
}